{
  "gene": "UniProtKB:A6NC98",
  "gene_symbol": "CCDC88B",
  "gene_name": "Coiled-coil domain-containing protein 88B",
  "term_id": "GO:0030705",
  "term_label": "cytoskeleton-dependent intracellular transport"
}